{
  "term_id": "GO:0032870",
  "gene": "UniProtKB:Q8TCW9",
  "gene_symbol": "PROKR1",
  "term_label": "cellular response to hormone stimulus",
  "gene_name": "Prokineticin receptor 1"
}